keratan sulfate-I proteoglycan biosynthetic process [GO:0140263] (biological process) Relationships: is a type of GO:0006487; is_a keratan sulfate proteoglycan biosynthetic process [GO:0018146] References: PMID:29340594 Definition: The chemical reactions and pathways resulting in the formation of keratan sulfate I (KS-I), N-linked via a GlcNAc attached to an asparigine residue in the target protein. Also known as: N-linked GlcNac-keratan sulfate-I proteoglycan biosynthetic process